{
  "gene_symbol": "HSPE1",
  "term_label": "mitochondrion",
  "gene_name": "10 kDa heat shock protein, mitochondrial",
  "term_id": "GO:0005739",
  "gene": "UniProtKB:P61604"
}